{
  "gene": "UniProtKB:Q8N2I2",
  "term_id": "GO:0005634",
  "term_label": "nucleus",
  "gene_name": "Zinc finger protein 619",
  "gene_symbol": "ZNF619"
}